{
  "term_label": "Unknown molecular function",
  "gene": "UniProtKB:Q9UD71",
  "gene_name": "Protein phosphatase 1 regulatory subunit 1B",
  "term_id": "UNKNOWN:0001",
  "gene_symbol": "PPP1R1B"
}